{
  "gene_name": "Phosphatidylinositol 4-phosphate 3-kinase C2 domain-containing subunit beta",
  "term_id": "GO:0035005",
  "gene": "UniProtKB:O00750",
  "term_label": "1-phosphatidylinositol-4-phosphate 3-kinase activity",
  "gene_symbol": "PIK3C2B"
}